{
  "gene_symbol": "SHARPIN",
  "term_label": "ubiquitin-protein transferase activity",
  "term_id": "GO:0004842",
  "gene": "UniProtKB:Q9H0F6",
  "gene_name": "Sharpin"
}